{
  "term_id": "GO:0005634",
  "term_label": "nucleus",
  "gene_name": "Transcription factor SOX-10",
  "gene": "UniProtKB:P56693",
  "gene_symbol": "SOX10"
}